{
  "term_label": "enzyme binding",
  "gene": "UniProtKB:Q9HAW7",
  "term_id": "GO:0019899",
  "gene_symbol": "UGT1A7",
  "gene_name": "UDP-glucuronosyltransferase 1A7"
}